skeletal muscle myosin thick filament assembly [GO:0030241] (biological process) Sources: GOC:ef, GOC:mah, GOC:mtg_muscle Definition: The aggregation, arrangement and bonding together of proteins to form the myosin-based thick filaments of myofibrils in skeletal muscle. Relationships: is_a striated muscle myosin thick filament assembly [GO:0071688]; is part of skeletal myofibril assembly [GO:0014866]